{
  "gene_name": "Rab-interacting lysosomal protein",
  "term_label": "cilium assembly",
  "term_id": "GO:0060271",
  "gene": "UniProtKB:Q96NA2",
  "gene_symbol": "RILP"
}